{
  "term_label": "plasma membrane",
  "gene_symbol": "NTRK2",
  "gene": "UniProtKB:Q16620",
  "gene_name": "BDNF_NT-3 growth factors receptor",
  "term_id": "GO:0005886"
}